lactate transmembrane transport [GO:0035873] (biological process) Also known as: lactate membrane transport Definition: The process in which lactate is transported across a membrane. Lactate is 2-hydroxypropanoate, CH3-CHOH-COOH; L(+)-lactate is formed by anaerobic glycolysis in animal tissues, and DL-lactate is found in sour milk, molasses and certain fruit juices. Note: Note that this term is not intended for use in annotating lateral movement within membranes. Subtypes: plasma membrane lactate transport [GO:0035879] Relationships: is a type of lactate transport [GO:0015727]; is a type of carboxylic acid transmembrane transport [GO:1905039] Sources: GOC:mcc, ISBN:0198506732